{
  "term_label": "synapse",
  "gene_symbol": "CHRNB3",
  "gene": "UniProtKB:Q05901",
  "term_id": "GO:0045202",
  "gene_name": "Neuronal acetylcholine receptor subunit beta-3"
}